positive regulation of beta-galactosidase activity [GO:1903771] (biological process) Definition: Any process that activates or increases the frequency, rate or extent of beta-galactosidase activity. Relationships: is a type of positive regulation of hydrolase activity [GO:0051345]; positively regulates beta-galactosidase activity [GO:0004565] References: PMID:11927518 Sources: GOC:BHF, GOC:TermGenie, GOC:nc, GO_REF:0000059 Also known as: positive regulation of beta-D-galactanase activity, positive regulation of beta-D-galactoside galactohydrolase activity, positive regulation of beta-D-lactosidase activity, positive regulation of beta-lactosidase activity, positive regulation of exo-(1->4)-beta-D-galactanase activity, positive regulation of trilactase activity, up regulation of beta-D-galactanase activity, up regulation of beta-D-galactoside galactohydrolase activity, up regulation of beta-D-lactosidase activity, up regulation of beta-galactosidase activity, up regulation of beta-lactosidase activity, up regulation of exo-(1->4)-beta-D-galactanase activity, up regulation of trilactase activity, up-regulation of beta-D-galactanase activity, up-regulation of beta-D-galactoside galactohydrolase activity, up-regulation of beta-D-lactosidase activity, up-regulation of beta-galactosidase activity, up-regulation of beta-lactosidase activity, up-regulation of exo-(1->4)-beta-D-galactanase activity, up-regulation of trilactase activity, upregulation of beta-D-galactanase activity, upregulation of beta-D-galactoside galactohydrolase activity, upregulation of beta-D-lactosidase activity, upregulation of beta-galactosidase activity, upregulation of beta-lactosidase activity, upregulation of exo-(1->4)-beta-D-galactanase activity, upregulation of trilactase activity, activation of beta-D-galactanase activity, activation of beta-D-galactoside galactohydrolase activity, activation of beta-D-lactosidase activity, activation of beta-galactosidase activity, activation of beta-lactosidase activity, activation of exo-(1->4)-beta-D-galactanase activity, activation of trilactase activity, activation of S 2107, activation of hydrolact, activation of lactose hydrolysis, activation of lactozym, activation of maxilact, activation of oryzatym, activation of sumiklat, positive regulation of S 2107, positive regulation of hydrolact, positive regulation of lactose hydrolysis, positive regulation of lactozym, positive regulation of maxilact, positive regulation of oryzatym, positive regulation of sumiklat, up regulation of S 2107, up regulation of hydrolact, up regulation of lactose hydrolysis, up regulation of lactozym, up regulation of maxilact, up regulation of oryzatym, up regulation of sumiklat, up-regulation of S 2107, up-regulation of hydrolact, up-regulation of lactose hydrolysis, up-regulation of lactozym, up-regulation of maxilact, up-regulation of oryzatym, up-regulation of sumiklat, upregulation of S 2107, upregulation of hydrolact, upregulation of lactose hydrolysis, upregulation of lactozym, upregulation of maxilact, upregulation of oryzatym, upregulation of sumiklat